{
  "term_label": "Unknown cellular component",
  "gene_name": "Voltage-gated purine nucleotide uniporter SLC17A9",
  "gene": "UniProtKB:Q9BYT1",
  "term_id": "UNKNOWN:0003",
  "gene_symbol": "SLC17A9"
}